axonal transport of messenger ribonucleoprotein complex [GO:0099088] (biological process) References: PMID:26586091 Sources: GOC:dos Also known as: axonal transport of mRNA RNP complex Definition: The directed movement of a messenger ribonucleoprotein complex along microtubules in axons. Relationships: is a type of GO:0098930